{
  "gene_name": "Histone H2B type 1-C_E_F_G_I",
  "term_label": "antimicrobial humoral immune response mediated by antimicrobial peptide",
  "gene": "UniProtKB:P62807",
  "gene_symbol": "H2BC10",
  "term_id": "GO:0061844"
}